{
  "gene_symbol": "LINC00301",
  "gene_name": "Putative uncharacterized protein encoded by LINC00301",
  "gene": "UniProtKB:Q8NCQ3",
  "term_id": "UNKNOWN:0003",
  "term_label": "Unknown cellular component"
}